{
  "gene_symbol": "APOE",
  "term_label": "high-density lipoprotein particle",
  "gene_name": "Apolipoprotein E",
  "term_id": "GO:0034364",
  "gene": "UniProtKB:P02649"
}